{
  "term_label": "RNA polymerase II cis-regulatory region sequence-specific DNA binding",
  "gene_name": "Zinc finger protein 595",
  "gene_symbol": "ZNF595",
  "gene": "UniProtKB:Q8IYB9",
  "term_id": "GO:0000978"
}